{
  "gene_name": "Testis-specific Y-encoded protein 8",
  "term_label": "chromatin binding",
  "gene": "UniProtKB:P0CW00",
  "gene_symbol": "TSPY8",
  "term_id": "GO:0003682"
}